LBD domain binding [GO:0050693] (molecular function) Also known as: ligand binding domain binding References: PMID:9682036 Definition: Binding to a protein's ligand binding domain (LBD) domain, found in nuclear receptors. In general, the LBDs consist of three layers comprised of twelve alpha-helices and several beta-strands that are organized around a lipophilic ligand-binding pocket. Relationships: is a type of protein domain specific binding [GO:0019904]